{
  "gene": "UniProtKB:O60879",
  "term_label": "actin filament polymerization",
  "gene_symbol": "DIAPH2",
  "gene_name": "Protein diaphanous homolog 2",
  "term_id": "GO:0030041"
}